{
  "term_label": "Unknown biological process",
  "gene_symbol": "A0A0G2JKW9",
  "gene": "UniProtKB:A0A0G2JKW9",
  "gene_name": "Uncharacterized protein",
  "term_id": "UNKNOWN:0002"
}